{
  "term_id": "GO:0001580",
  "gene": "UniProtKB:Q9NYV8",
  "gene_symbol": "TAS2R14",
  "term_label": "detection of chemical stimulus involved in sensory perception of bitter taste",
  "gene_name": "Taste receptor type 2 member 14"
}